{
  "term_label": "nucleus",
  "gene_symbol": "CAMTA1",
  "gene_name": "Calmodulin-binding transcription activator 1",
  "term_id": "GO:0005634",
  "gene": "UniProtKB:Q9Y6Y1"
}